{
  "gene": "UniProtKB:Q8N239",
  "term_label": "Unknown cellular component",
  "gene_name": "Kelch-like protein 34",
  "gene_symbol": "KLHL34",
  "term_id": "UNKNOWN:0003"
}